nuclear receptor-mediated mineralocorticoid signaling pathway [GO:0031959] (biological process) Definition: A nuclear receptor-mediated signaling pathway initiated by a mineralocorticoid binding to an intracellular receptor of the nuclear receptor protein family, and ending with regulation of a downstream cellular process, e.g. transcription. References: PMID:11027914, PMID:12606724, PMID:15240347 Also known as: mineralocorticoid receptor signaling pathway, mineralocorticoid receptor signalling pathway, intracellular mineralocorticoid receptor signaling pathway Relationships: is a type of nuclear receptor-mediated corticosteroid signaling pathway [GO:0031958]